{
  "gene": "UniProtKB:Q13444",
  "term_label": "extracellular space",
  "term_id": "GO:0005615",
  "gene_name": "Disintegrin and metalloproteinase domain-containing protein 15",
  "gene_symbol": "ADAM15"
}